{
  "gene_symbol": "GPR6",
  "term_label": "plasma membrane",
  "gene_name": "G-protein coupled receptor 6",
  "gene": "UniProtKB:P46095",
  "term_id": "GO:0005886"
}